negative regulation of steroid metabolic process [GO:0045939] (biological process) Definition: Any process that stops, prevents, or reduces the frequency, rate or extent of the chemical reactions and pathways involving steroids. Sources: GOC:go_curators Also known as: down regulation of steroid metabolic process, down-regulation of steroid metabolic process, downregulation of steroid metabolic process, negative regulation of steroid metabolism, inhibition of steroid metabolic process Relationships: is a type of regulation of steroid metabolic process [GO:0019218]; is a type of negative regulation of lipid metabolic process [GO:0045833]; negatively regulates GO:0008202 Subtypes: GO:0010894, GO:0031950, negative regulation of cholesterol metabolic process [GO:0090206]